adenine metabolic process [GO:0046083] (biological process) Definition: The chemical reactions and pathways involving adenine, 6-aminopurine, one of the five main bases found in nucleic acids and a component of numerous important derivatives of its corresponding ribonucleoside, adenosine. Subtypes: adenine catabolic process [GO:0006146], adenine biosynthetic process [GO:0046084] Sources: GOC:go_curators Relationships: is a type of purine nucleobase metabolic process [GO:0006144] Also known as: adenine metabolism